type 1 orexin receptor binding [GO:0031771] (MF) Definition: Binding to a type 1 orexin receptor. Sources: GOC:mah, GOC:nln Also known as: OX1 orexin receptor binding, type 1 hypocretin receptor binding, type 1 hypocretin receptor ligand Relationships: is a type of GO:0042324